{
  "term_id": "GO:0048025",
  "term_label": "negative regulation of mRNA splicing, via spliceosome",
  "gene": "UniProtKB:P57723",
  "gene_symbol": "PCBP4",
  "gene_name": "Poly(rC)-binding protein 4"
}